{
  "term_label": "DNA-binding transcription factor activity, RNA polymerase II-specific",
  "gene_name": "Mesoderm posterior protein 2",
  "gene_symbol": "MESP2",
  "term_id": "GO:0000981",
  "gene": "UniProtKB:Q0VG99"
}